(1-hydroxycyclohexan-1-yl)acetyl-CoA lyase activity [GO:0047446] (molecular function) Also known as: (1-hydroxycyclohexan-1-yl)acetyl-CoA cyclohexanone-lyase (acetyl-CoA-forming), (1-hydroxycyclohexan-1-yl)acetyl-CoA cyclohexanone-lyase activity Definition: Catalysis of the reaction: (1-hydroxycyclohexan-1-yl)acetyl-CoA = acetyl-CoA + cyclohexanone. Sources: EC:4.1.3.35, RHEA:23868 Relationships: is a type of oxo-acid-lyase activity [GO:0016833]